{
  "term_id": "GO:0005814",
  "gene": "UniProtKB:Q6UVJ0",
  "gene_symbol": "SASS6",
  "gene_name": "Spindle assembly abnormal protein 6 homolog",
  "term_label": "centriole"
}